{
  "term_label": "adaptive immune response",
  "term_id": "GO:0002250",
  "gene": "UniProtKB:P01569",
  "gene_name": "Interferon alpha-5",
  "gene_symbol": "IFNA5"
}